{
  "term_id": "GO:1901856",
  "term_label": "negative regulation of cellular respiration",
  "gene_symbol": "ETFRF1",
  "gene_name": "Electron transfer flavoprotein regulatory factor 1",
  "gene": "UniProtKB:Q6IPR1"
}